nuclear inner membrane [GO:0005637] (cellular component) Definition: The inner, i.e. lumen-facing, lipid bilayer of the nuclear envelope. Sources: GOC:ma Relationships: is a type of organelle inner membrane [GO:0019866]; is a type of GO:0031965 Also known as: inner envelope, inner nuclear membrane, nucleus inner membrane